{
  "gene_symbol": "ETDA",
  "term_label": "Unknown cellular component",
  "gene_name": "Embryonic testis differentiation protein homolog A",
  "gene": "UniProtKB:Q3ZM63",
  "term_id": "UNKNOWN:0003"
}